{
  "gene_symbol": "VCAM1",
  "gene_name": "Vascular cell adhesion protein 1",
  "term_id": "GO:0005178",
  "gene": "UniProtKB:P19320",
  "term_label": "integrin binding"
}